{
  "term_label": "action potential",
  "gene": "UniProtKB:Q9UIX4",
  "gene_symbol": "KCNG1",
  "gene_name": "Potassium voltage-gated channel subfamily G member 1",
  "term_id": "GO:0001508"
}